{
  "gene": "UniProtKB:P0CH98",
  "term_id": "UNKNOWN:0002",
  "gene_symbol": "FAM106C",
  "term_label": "Unknown biological process",
  "gene_name": "Protein FAM106C"
}